{
  "gene": "UniProtKB:P17026",
  "term_label": "Unknown molecular function",
  "term_id": "UNKNOWN:0001",
  "gene_name": "Zinc finger protein 22",
  "gene_symbol": "ZNF22"
}